{
  "gene": "UniProtKB:Q13461",
  "gene_name": "Forkhead box protein E3",
  "term_label": "anatomical structure morphogenesis",
  "term_id": "GO:0009653",
  "gene_symbol": "FOXE3"
}